{
  "gene_name": "Complement factor H-related protein 2",
  "term_label": "extracellular space",
  "term_id": "GO:0005615",
  "gene_symbol": "CFHR2",
  "gene": "UniProtKB:P36980"
}